{
  "gene": "UniProtKB:Q6MZT1",
  "term_label": "Unknown molecular function",
  "gene_symbol": "RGS7BP",
  "term_id": "UNKNOWN:0001",
  "gene_name": "Regulator of G-protein signaling 7-binding protein"
}